{
  "term_label": "protein tyrosine phosphatase activity",
  "term_id": "GO:0004725",
  "gene": "UniProtKB:P30304",
  "gene_name": "M-phase inducer phosphatase 1",
  "gene_symbol": "CDC25A"
}